{
  "gene": "UniProtKB:Q11206",
  "gene_symbol": "ST3GAL4",
  "term_id": "UNKNOWN:0003",
  "term_label": "Unknown cellular component",
  "gene_name": "CMP-N-acetylneuraminate-beta-galactosamide-alpha-2,3-sialyltransferase 4"
}